{
  "gene": "UniProtKB:Q6UW49",
  "term_id": "GO:0007340",
  "gene_name": "Sperm equatorial segment protein 1",
  "gene_symbol": "SPESP1",
  "term_label": "acrosome reaction"
}